(2E,6E)-farnesyl diphosphate synthase activity [GO:0004337] (molecular function) Sources: RHEA:19361 Definition: Catalysis of the reaction: (2E)-geranyl diphosphate + isopentenyl diphosphate = (2E,6E)-farnesyl diphosphate + diphosphate. Relationships: is a type of prenyl diphosphate synthase activity [GO:0120531] Note: Note that this is the second step in the formation of farnesyl diphosphate. The first step is 'dimethylallyltransferase activity ; GO:0004161'. Consider also annotating to the biological process term 'farnesyl diphosphate biosynthetic process ; GO:0045337'. Also known as: farnesyl diphosphate synthase activity, farnesyl pyrophosphate synthetase activity, farnesyl-diphosphate synthase activity, geranyltranstransferase activity, FPP synthetase activity, farnesyl diphosphate synthetase activity, farnesylpyrophosphate synthetase activity, geranyl transferase I, geranyl-diphosphate:isopentenyl-diphosphate geranyltranstransferase activity, geranyltransferase activity